{
  "term_label": "cGMP catabolic process",
  "gene_name": "High affinity cGMP-specific 3',5'-cyclic phosphodiesterase 9A",
  "term_id": "GO:0046069",
  "gene": "UniProtKB:O76083",
  "gene_symbol": "PDE9A"
}